{
  "gene_name": "Frataxin, mitochondrial",
  "term_label": "iron chaperone activity",
  "gene_symbol": "FXN",
  "term_id": "GO:0034986",
  "gene": "UniProtKB:Q16595"
}